{
  "term_label": "Unknown cellular component",
  "gene_symbol": "TSKU",
  "gene": "UniProtKB:Q8WUA8",
  "gene_name": "Tsukushi",
  "term_id": "UNKNOWN:0003"
}